{
  "term_id": "GO:0005886",
  "term_label": "plasma membrane",
  "gene_symbol": "SLC5A1",
  "gene": "UniProtKB:P13866",
  "gene_name": "Sodium_glucose cotransporter 1"
}